{
  "gene_name": "LIM domain and actin-binding protein 1",
  "term_label": "actin filament binding",
  "gene_symbol": "LIMA1",
  "gene": "UniProtKB:Q9UHB6",
  "term_id": "GO:0051015"
}